{
  "gene_name": "Netrin receptor UNC5A",
  "gene": "UniProtKB:Q6ZN44",
  "gene_symbol": "UNC5A",
  "term_label": "Unknown cellular component",
  "term_id": "UNKNOWN:0003"
}